{
  "gene_symbol": "CCN1",
  "term_label": "heparin binding",
  "gene_name": "CCN family member 1",
  "gene": "UniProtKB:O00622",
  "term_id": "GO:0008201"
}